{
  "term_id": "GO:0007155",
  "gene_symbol": "PCDHGA8",
  "term_label": "cell adhesion",
  "gene_name": "Protocadherin gamma-A8",
  "gene": "UniProtKB:Q9Y5G5"
}